{
  "term_label": "phosphatidylinositol-mediated signaling",
  "gene_name": "Phosphatidylinositol 4-kinase beta",
  "gene_symbol": "PI4KB",
  "gene": "UniProtKB:Q9UBF8",
  "term_id": "GO:0048015"
}